{
  "gene": "UniProtKB:Q12879",
  "term_label": "long-term synaptic potentiation",
  "term_id": "GO:0060291",
  "gene_symbol": "GRIN2A",
  "gene_name": "Glutamate receptor ionotropic, NMDA 2A"
}